venom-mediated inhibition of high voltage-gated calcium channel activity [GO:0044475] (biological process) References: PMID:20920515 Sources: GOC:fj, GOC:jl Relationships: is a type of GO:0044474 Also known as: envenomation resulting in negative regulation of high voltage-gated calcium channel activity in another organism, envenomation resulting in negative regulation of high voltage-gated calcium channel activity in other organism Definition: A process in which an organism inhibits or disrupts the activity of a high voltage-gated calcium channel in another organism via the action of a venom.